{
  "gene": "UniProtKB:P14091",
  "gene_symbol": "CTSE",
  "gene_name": "Cathepsin E",
  "term_id": "GO:0004190",
  "term_label": "aspartic-type endopeptidase activity"
}